{
  "term_label": "cilium movement",
  "gene_name": "Nucleoside diphosphate kinase homolog 5",
  "gene_symbol": "NME5",
  "term_id": "GO:0003341",
  "gene": "UniProtKB:P56597"
}